{
  "gene_name": "Sperm mitochondrial-associated cysteine-rich protein",
  "term_label": "Unknown molecular function",
  "term_id": "UNKNOWN:0001",
  "gene_symbol": "SMCP",
  "gene": "UniProtKB:P49901"
}